galactose 1-dehydrogenase activity [GO:0019151] (molecular function) Relationships: is a type of GO:0016616 Sources: EC:1.1.1.48 Also known as: D-galactose 1-dehydrogenase activity, D-galactose dehydrogenase activity, D-galactose:NAD+ 1-oxidoreductase activity, NAD-dependent D-galactose dehydrogenase activity, beta-galactose dehydrogenase activity Definition: Catalysis of the reaction: D-galactose + NAD+ = D-galactono-1,4-lactone + NADH + H+.